{
  "gene_name": "Double homeobox protein 4-like protein 7",
  "gene": "UniProtKB:P0CJ90",
  "term_label": "nucleus",
  "term_id": "GO:0005634",
  "gene_symbol": "DUX4L7"
}